{
  "gene": "UniProtKB:Q14656",
  "term_id": "UNKNOWN:0002",
  "gene_symbol": "TMEM187",
  "gene_name": "Transmembrane protein 187",
  "term_label": "Unknown biological process"
}